{
  "term_id": "GO:0005634",
  "gene_name": "Zinc finger protein GLI2",
  "gene": "UniProtKB:P10070",
  "term_label": "nucleus",
  "gene_symbol": "GLI2"
}